{
  "gene": "UniProtKB:Q8NG84",
  "gene_symbol": "OR2AK2",
  "gene_name": "Olfactory receptor 2AK2",
  "term_label": "plasma membrane",
  "term_id": "GO:0005886"
}